{
  "gene": "UniProtKB:O75610",
  "term_label": "cytokine activity",
  "gene_symbol": "LEFTY1",
  "gene_name": "Left-right determination factor 1",
  "term_id": "GO:0005125"
}